calcium oxalate binding [GO:0046904] (molecular function) Definition: Binding to calcium oxalate, CaC2O4, a salt of oxalic acid. In animals, it may be excreted in urine or retained in the form of urinary calculi. Relationships: is a type of carboxylic acid binding [GO:0031406] Sources: ISBN:0721662544